positive regulation of sporocarp development involved in sexual reproduction [GO:1902060] (biological process) Also known as: activation of fruiting body development involved in sexual reproduction, activation of fruiting body formation involved in sexual reproduction, positive regulation of fruiting body development involved in sexual reproduction, positive regulation of fruiting body formation involved in sexual reproduction, up regulation of fruiting body development involved in sexual reproduction, up regulation of fruiting body formation involved in sexual reproduction, up-regulation of fruiting body development involved in sexual reproduction, up-regulation of fruiting body formation involved in sexual reproduction, upregulation of fruiting body development involved in sexual reproduction, upregulation of fruiting body formation involved in sexual reproduction, up regulation of sporocarp development involved in sexual reproduction, up-regulation of sporocarp development involved in sexual reproduction, upregulation of sporocarp development involved in sexual reproduction, activation of ascus development, activation of perfect stage fruiting body development, activation of sporocarp development involved in sexual reproduction, positive regulation of ascus development, positive regulation of perfect stage fruiting body development, up regulation of ascus development, up regulation of perfect stage fruiting body development, up-regulation of ascus development, up-regulation of perfect stage fruiting body development, upregulation of ascus development, upregulation of perfect stage fruiting body development Definition: Any process that activates or increases the frequency, rate or extent of sporocarp development involved in sexual reproduction. Subtypes: positive regulation of cleistothecium development [GO:0070798] Relationships: is a type of GO:0075261; is a type of regulation of sporocarp development involved in sexual reproduction [GO:1902058]; positively regulates sporocarp development involved in sexual reproduction [GO:0000909] References: PMID:23480775 Sources: GOC:TermGenie, GOC:di